novofumigatonin biosynthetic process [GO:0140782] (biological process) Also known as: novofumigatonin anabolism, novofumigatonin biosynthesis, novofumigatonin formation, novofumigatonin synthesis Definition: The chemical reactions and pathways resulting in the formation of novofumigatonin, a heavily oxygenated meroterpenoid containing a unique orthoester moiety. Relationships: is_a terpenoid biosynthetic process [GO:0016114]; is a type of ketone biosynthetic process [GO:0042181] References: PMID:29968715